regulation of siRNA processing [GO:0070921] (biological process) Sources: GOC:mah Definition: Any process that modulates the frequency, rate or extent of siRNA processing. Subtypes: negative regulation of siRNA processing [GO:1903704], positive regulation of siRNA processing [GO:1903705] Also known as: regulation of RNA interference, production of siRNA, regulation of chromatin silencing by small RNA, production of siRNA, regulation of production of siRNA involved in RNA interference, regulation of production of siRNA involved in chromatin silencing by small RNA, regulation of production of siRNA involved in PTGS, regulation of production of siRNA involved in gene silencing by small RNA, regulation of production of siRNA involved in post-transcriptional gene silencing by RNA, regulation of siRNA production Relationships: is a type of regulation of regulatory ncRNA processing [GO:0070920]; regulates GO:0030422